negative regulation of low-density lipoprotein particle receptor catabolic process [GO:0032804] (biological process) Sources: GOC:mah Relationships: is a type of GO:0032803; is a type of GO:0042177; is_a negative regulation of receptor catabolic process [GO:2000645]; negatively regulates low-density lipoprotein particle receptor catabolic process [GO:0032802] Definition: Any process that stops, prevents, or reduces the frequency, rate or extent of the chemical reactions and pathways resulting in the breakdown of low-density lipoprotein receptors. Also known as: down regulation of low-density lipoprotein receptor catabolic process, down-regulation of low-density lipoprotein receptor catabolic process, downregulation of low-density lipoprotein receptor catabolic process, negative regulation of low-density lipoprotein receptor breakdown, negative regulation of low-density lipoprotein receptor catabolic process, negative regulation of low-density lipoprotein receptor catabolism, negative regulation of low-density lipoprotein receptor degradation, inhibition of low-density lipoprotein receptor catabolic process